{
  "term_id": "GO:0006906",
  "gene": "UniProtKB:O95249",
  "gene_symbol": "GOSR1",
  "gene_name": "Golgi SNAP receptor complex member 1",
  "term_label": "vesicle fusion"
}